D-alanine-(R)-lactate ligase activity [GO:0160220] (molecular function) Definition: Catalysis of the reaction: (R)-lactate + ATP + D-alanine = ADP + D-alanyl-(R)-lactate + phosphate. Sources: RHEA:37347 Also known as: D-alanyl-D-lactate ligase activity Relationships: is a type of ligase activity, forming carbon-oxygen bonds [GO:0016875]